negative regulation of ubiquitin-protein transferase activity [GO:0051444] (biological process) Relationships: is a type of negative regulation of protein ubiquitination [GO:0031397]; is_a negative regulation of catalytic activity [GO:0043086]; is a type of GO:0051438; negatively regulates ubiquitin-protein transferase activity [GO:0004842] Definition: Any process that stops, prevents, or reduces the frequency, rate or extent of ubiquitin transferase activity. Subtypes: negative regulation of ubiquitin protein ligase activity [GO:1904667] Also known as: down regulation of ubiquitin transferase activity, down-regulation of ubiquitin transferase activity, downregulation of ubiquitin transferase activity, negative regulation of ubiquitin transferase activity, APC inhibition, APC inhibitor, SCF complex inhibitor, anaphase promoting complex inhibition, anaphase promoting complex inhibitor, anaphase-promoting complex inhibition, anaphase-promoting complex inhibitor, inhibition of ubiquitin transferase activity, ubiquitin transferase inhibitor Sources: GOC:ai, GOC:tb